{
  "gene_symbol": "PAQR3",
  "term_id": "UNKNOWN:0001",
  "gene": "UniProtKB:Q6TCH7",
  "term_label": "Unknown molecular function",
  "gene_name": "Progestin and adipoQ receptor family member 3"
}